{
  "term_label": "RNA polymerase II cis-regulatory region sequence-specific DNA binding",
  "gene_name": "Homeobox protein Hox-B7",
  "gene_symbol": "HOXB7",
  "term_id": "GO:0000978",
  "gene": "UniProtKB:P09629"
}